glutamatergic neuron differentiation [GO:1905962] (biological process) Relationships: is a type of neuron differentiation [GO:0030182] Subtypes: cerebellar granule cell differentiation [GO:0021707], retinal bipolar neuron differentiation [GO:0060040] References: PMID:24030726 Sources: GOC:TermGenie, GO_REF:0000086 Regulation: regulated by regulation of glutamatergic neuron differentiation [GO:0120006]; negatively regulated by negative regulation of glutamatergic neuron differentiation [GO:0120007]; positively regulated by positive regulation of glutamatergic neuron differentiation [GO:0120008] Definition: The process in which a relatively unspecialized cell acquires the specialized features of a glutamatergic neuron.